{
  "gene_symbol": "CALCRL",
  "term_label": "adenylate cyclase-activating G protein-coupled receptor signaling pathway",
  "gene": "UniProtKB:Q16602",
  "gene_name": "Calcitonin gene-related peptide type 1 receptor",
  "term_id": "GO:0007189"
}